{
  "gene_name": "Beclin-2",
  "term_label": "protein-macromolecule adaptor activity",
  "term_id": "GO:0030674",
  "gene": "UniProtKB:A8MW95",
  "gene_symbol": "BECN2"
}